sodium channel complex [GO:0034706] (cellular component) Definition: An ion channel complex through which sodium ions pass. Sources: GOC:mah Relationships: is a type of cation channel complex [GO:0034703] Subtypes: voltage-gated sodium channel complex [GO:0001518], kainate selective glutamate receptor complex [GO:0032983]